{
  "gene_name": "Beta-hexosaminidase subunit alpha",
  "term_id": "GO:0016020",
  "gene": "UniProtKB:P06865",
  "term_label": "membrane",
  "gene_symbol": "HEXA"
}